{
  "term_id": "GO:0051225",
  "term_label": "spindle assembly",
  "gene_name": "HAUS augmin-like complex subunit 7",
  "gene_symbol": "HAUS7",
  "gene": "UniProtKB:Q99871"
}